{
  "gene_name": "GS homeobox 1",
  "term_id": "GO:0030182",
  "gene_symbol": "GSX1",
  "gene": "UniProtKB:Q9H4S2",
  "term_label": "neuron differentiation"
}